{
  "term_label": "cell surface",
  "gene_symbol": "DCC",
  "term_id": "GO:0009986",
  "gene": "UniProtKB:P43146",
  "gene_name": "Netrin receptor DCC"
}